{
  "gene": "UniProtKB:Q9BVA1",
  "term_id": "GO:0005200",
  "gene_symbol": "TUBB2B",
  "gene_name": "Tubulin beta-2B chain",
  "term_label": "structural constituent of cytoskeleton"
}